acetate:monoatomic cation symporter activity [GO:0043893] (molecular function) Definition: Enables the transfer of acetate from one side of a membrane to the other according to the reaction: acetate(out) + cation(out) = acetate(in) + cation(in). Also known as: acetate permease, acetate:cation symporter activity, acetate-cation symporter activity, acetate/cation symporter activity, cation-acetate symporter activity, cation/acetate symporter activity, cation:acetate symporter activity, ActP References: PMID:14563880 Sources: GOC:jl Relationships: is a type of GO:0015123; is a type of solute:monoatomic cation symporter activity [GO:0015294]; is a type of secondary active monocarboxylate transmembrane transporter activity [GO:0015355] Subtypes: acetate:proton symporter activity [GO:0015360]